{
  "term_id": "GO:0042105",
  "gene_name": "T-cell surface glycoprotein CD3 zeta chain",
  "gene_symbol": "CD247",
  "gene": "UniProtKB:P20963",
  "term_label": "alpha-beta T cell receptor complex"
}